{
  "term_id": "GO:0048407",
  "gene": "UniProtKB:P16234",
  "gene_name": "Platelet-derived growth factor receptor alpha",
  "term_label": "platelet-derived growth factor binding",
  "gene_symbol": "PDGFRA"
}